{
  "gene": "UniProtKB:O75306",
  "gene_name": "NADH dehydrogenase [ubiquinone] iron-sulfur protein 2, mitochondrial",
  "term_id": "GO:0006120",
  "term_label": "mitochondrial electron transport, NADH to ubiquinone",
  "gene_symbol": "NDUFS2"
}